{
  "term_id": "GO:0070743",
  "term_label": "interleukin-23 complex",
  "gene": "UniProtKB:Q9NPF7",
  "gene_symbol": "IL23A",
  "gene_name": "Interleukin-23 subunit alpha"
}